negative regulation of basophil degranulation [GO:1903582] (biological process) Relationships: is a type of negative regulation of myeloid leukocyte mediated immunity [GO:0002887]; is a type of GO:0043301; is a type of GO:0050777; is a type of regulation of basophil degranulation [GO:1903581]; negatively regulates GO:0002561 References: PMID:10880837 Sources: GOC:TermGenie, GO_REF:0000058 Definition: Any process that stops, prevents or reduces the frequency, rate or extent of basophil degranulation. Also known as: down regulation of basophil degranulation, down-regulation of basophil degranulation, downregulation of basophil degranulation, inhibition of basophil degranulation